yeast-form cell wall [GO:0030445] (cellular component) Relationships: is a type of fungal-type cell wall [GO:0009277] Sources: GOC:mah, GOC:mcc Note: See also the Fungal Anatomy Ontology term 'vegetative cell ; FAO:0000032'. Definition: The wall surrounding a cell of a dimorphic fungus growing in the single-cell budding yeast form, in contrast to the filamentous or hyphal form.